acetyldiaminopimelate aminotransferase activity [GO:0043760] (molecular function) Definition: Catalysis of the reaction: N-acetyl-L-2,6-diaminoheptanedioate + 2-oxoglutarate = N-acetyl-2-L-amino-6-oxoheptanedioate + L-glutamate. Also known as: N-acetyl-L,L-diaminopimelate aminotransferase activity, N-acetyl-diaminopimelate aminotransferase activity Relationships: is a type of transaminase activity [GO:0008483] References: PMID:1906065